{
  "term_label": "Unknown cellular component",
  "gene": "UniProtKB:Q9HAH7",
  "gene_name": "Probable fibrosin-1",
  "term_id": "UNKNOWN:0003",
  "gene_symbol": "FBRS"
}